positive regulation of neutrophil migration [GO:1902624] (BP) References: PMID:1826836 Sources: GOC:TermGenie, GO_REF:0000058 Also known as: up regulation of neutrophil migration, up-regulation of neutrophil migration, upregulation of neutrophil migration, activation of neutrophil migration Subtypes: positive regulation of neutrophil chemotaxis [GO:0090023], positive regulation of neutrophil extravasation [GO:2000391] Relationships: is a type of positive regulation of leukocyte migration [GO:0002687]; is a type of regulation of neutrophil migration [GO:1902622]; positively regulates GO:1990266 Definition: Any process that activates or increases the frequency, rate or extent of neutrophil migration.